{
  "gene_symbol": "MUTYH",
  "gene_name": "Adenine DNA glycosylase",
  "term_label": "adenine/guanine mispair binding",
  "term_id": "GO:0035485",
  "gene": "UniProtKB:Q9UIF7"
}